uridine transmembrane transport [GO:0015862] (biological process) Definition: The directed movement of uridine, uracil riboside, across a lipid bilayer, by means of some agent such as a transporter or pore. Relationships: is a type of GO:0015864; is a type of GO:0072531; is a type of nucleoside transmembrane transport [GO:1901642] Sources: GOC:go_curators